{
  "term_id": "GO:0009115",
  "gene": "UniProtKB:P47989",
  "term_label": "xanthine catabolic process",
  "gene_name": "Xanthine dehydrogenase_oxidase",
  "gene_symbol": "XDH"
}